{
  "gene_symbol": "SPG11",
  "term_label": "cytoplasm",
  "gene_name": "Spatacsin",
  "gene": "UniProtKB:Q96JI7",
  "term_id": "GO:0005737"
}